{
  "term_label": "cytosol",
  "gene_name": "Fatty acid-binding protein 9",
  "gene": "UniProtKB:Q0Z7S8",
  "gene_symbol": "FABP9",
  "term_id": "GO:0005829"
}